{
  "term_id": "GO:0006357",
  "gene": "UniProtKB:Q96EG3",
  "gene_name": "Zinc finger protein 837",
  "gene_symbol": "ZNF837",
  "term_label": "regulation of transcription by RNA polymerase II"
}